5-hydroxy-6E,8Z,11Z,14Z-icosatetraenoic acid binding [GO:0050647] (molecular function) Sources: GOC:ai Also known as: 5-hydroxy-6E,8Z,11Z,14Z-eicosatetraenoic acid binding Relationships: is a type of long-chain fatty acid binding [GO:0036041]; is a type of icosanoid binding [GO:0050542]; is a type of fatty acid derivative binding [GO:1901567] Definition: Binding to 5-hydroxy-6E,8Z,11Z,14Z-icosatetraenoic acid, a straight-chain fatty acid with twenty carbon atoms and four double bonds.